{
  "gene_name": "Olfactory receptor 52D1",
  "gene_symbol": "OR52D1",
  "term_label": "olfactory receptor activity",
  "term_id": "GO:0004984",
  "gene": "UniProtKB:Q9H346"
}